intermediate filament polymerization or depolymerization [GO:0045105] (biological process) Sources: GOC:ai Definition: Assembly or disassembly of intermediate filaments by the addition or removal of component parts from a filament. Relationships: is a type of protein-containing complex organization [GO:0043933]; is part of GO:0045104 Subtypes: intermediate filament depolymerization [GO:0045106], intermediate filament polymerization [GO:0045107] Regulation: regulated by GO:0045108